{
  "term_id": "GO:0002757",
  "gene_name": "CMRF35-like molecule 5",
  "gene": "UniProtKB:Q6UXZ3",
  "gene_symbol": "CD300LD",
  "term_label": "immune response-activating signaling pathway"
}